{
  "gene": "UniProtKB:A0A0C4DH72",
  "gene_name": "Immunoglobulin kappa variable 1-6",
  "term_label": "immune response",
  "gene_symbol": "IGKV1-6",
  "term_id": "GO:0006955"
}